{
  "gene": "UniProtKB:A6NNX1",
  "term_label": "Unknown biological process",
  "gene_symbol": "RIIAD1",
  "gene_name": "RIIa domain-containing protein 1",
  "term_id": "UNKNOWN:0002"
}